{
  "term_label": "negative regulation of Notch signaling pathway",
  "gene_name": "RBPJ-interacting and tubulin-associated protein 1",
  "gene": "UniProtKB:Q96K30",
  "term_id": "GO:0045746",
  "gene_symbol": "RITA1"
}